{
  "gene_name": "Selenoprotein K",
  "term_id": "GO:0032469",
  "gene": "UniProtKB:Q9Y6D0",
  "gene_symbol": "SELENOK",
  "term_label": "endoplasmic reticulum calcium ion homeostasis"
}